protein serine pyrophosphorylase activity [GO:0141090] (molecular function) Definition: Catalysis of the reaction: protein phospho-serine + inositol 5-triphosphate pentakisphosphate = protein diphospho-serine + inositol 5-diphosphate pentakisphosphate. References: PMID:36603579 Sources: RHEA:64104 Also known as: protein serine pyrophosphatase activity Relationships: is a type of GO:0016776